{
  "gene_name": "T cell receptor alpha joining 21 (Fragment)",
  "term_label": "Unknown biological process",
  "gene": "UniProtKB:A0A075B6V2",
  "term_id": "UNKNOWN:0002",
  "gene_symbol": "TRAJ21"
}